{
  "term_label": "cilium assembly",
  "gene_symbol": "CEP250",
  "term_id": "GO:0060271",
  "gene": "UniProtKB:Q9BV73",
  "gene_name": "Centrosome-associated protein CEP250"
}